lipopeptide binding [GO:0071723] (molecular function) Definition: Binding to a lipopeptide, any of a group of organic compounds comprising two or more amino acids linked by peptide bonds and containing a nonprotein group consisting of a lipid or lipids. Relationships: is a type of lipid binding [GO:0008289]; is a type of amide binding [GO:0033218] References: PMID:12077222, PMID:12524386, PMID:2757794 Sources: GOC:add Note: Note that bacterial lipopeptides are derived from bacterial lipoproteins, but the two terms are sometimes used interchangeably in the literature. Subtypes: triacyl lipopeptide binding [GO:0042497], diacyl lipopeptide binding [GO:0042498] Also known as: bacterial lipopeptide binding, bacterial lipoprotein binding